{
  "gene_symbol": "PDHX",
  "gene": "UniProtKB:O00330",
  "term_id": "GO:0045254",
  "gene_name": "Pyruvate dehydrogenase protein X component, mitochondrial",
  "term_label": "pyruvate dehydrogenase complex"
}